{
  "term_id": "GO:0005634",
  "term_label": "nucleus",
  "gene_name": "Transcription factor E3",
  "gene": "UniProtKB:P19532",
  "gene_symbol": "TFE3"
}